amorphous vesicle [GO:1990006] (cellular component) Relationships: is a type of cytoplasmic vesicle [GO:0031410] Definition: A cytoplasmic membrane-bounded vesicle first described in dendrites, categorized by smooth membranes, electron-lucent interiors and irregular shapes. Sometimes occurs in clumps. Amorphous vesicles have been found to contain material taken up from the extracellular space, therefore suggesting that they may be part of the endosomal pathway. References: PMID:11896161 Sources: NIF_Subcellular:sao1531915298